{
  "gene": "UniProtKB:O15144",
  "term_id": "GO:0005885",
  "term_label": "Arp2/3 protein complex",
  "gene_symbol": "ARPC2",
  "gene_name": "Actin-related protein 2_3 complex subunit 2"
}